{
  "gene_symbol": "DNAAF5",
  "term_label": "dynein intermediate chain binding",
  "term_id": "GO:0045505",
  "gene": "UniProtKB:Q86Y56",
  "gene_name": "Dynein axonemal assembly factor 5"
}